{
  "gene_name": "Keratin, type I cytoskeletal 23",
  "gene_symbol": "KRT23",
  "term_label": "structural constituent of skin epidermis",
  "gene": "UniProtKB:Q9C075",
  "term_id": "GO:0030280"
}